{
  "term_id": "GO:0060090",
  "gene": "UniProtKB:P40305",
  "gene_name": "Interferon alpha-inducible protein 27, mitochondrial",
  "term_label": "molecular adaptor activity",
  "gene_symbol": "IFI27"
}